{
  "gene_name": "Serine_threonine-protein kinase BRSK2",
  "gene_symbol": "BRSK2",
  "term_label": "establishment of cell polarity",
  "term_id": "GO:0030010",
  "gene": "UniProtKB:Q8IWQ3"
}